regulation of glucagon secretion [GO:0070092] (biological process) Subtypes: GO:0070093, positive regulation of glucagon secretion [GO:0070094] Relationships: is a type of GO:0090276; regulates glucagon secretion [GO:0070091] Definition: Any process that modulates the frequency, rate or extent of the regulated release of glucagon. Sources: GOC:BHF, GOC:mah